{
  "gene": "UniProtKB:Q14118",
  "gene_name": "Dystroglycan 1",
  "term_label": "nerve development",
  "term_id": "GO:0021675",
  "gene_symbol": "DAG1"
}